{
  "gene": "UniProtKB:Q9NYY3",
  "term_label": "centrosome",
  "gene_name": "Serine_threonine-protein kinase PLK2",
  "term_id": "GO:0005813",
  "gene_symbol": "PLK2"
}